{
  "gene_symbol": "GM2A",
  "gene_name": "Ganglioside GM2 activator",
  "term_label": "ganglioside catabolic process",
  "gene": "UniProtKB:P17900",
  "term_id": "GO:0006689"
}